{
  "term_label": "cytoplasm",
  "gene_symbol": "LIX1",
  "gene_name": "Protein limb expression 1 homolog",
  "gene": "UniProtKB:Q8N485",
  "term_id": "GO:0005737"
}